{
  "gene_symbol": "RABIF",
  "gene_name": "Guanine nucleotide exchange factor MSS4",
  "term_id": "GO:0006892",
  "term_label": "post-Golgi vesicle-mediated transport",
  "gene": "UniProtKB:P47224"
}